{
  "gene_name": "Kinesin-like protein KIF9",
  "term_id": "GO:0005737",
  "gene_symbol": "KIF9",
  "gene": "UniProtKB:Q9HAQ2",
  "term_label": "cytoplasm"
}